{
  "gene_name": "Peroxisomal membrane protein 11C",
  "gene": "UniProtKB:Q96HA9",
  "gene_symbol": "PEX11G",
  "term_label": "peroxisome fission",
  "term_id": "GO:0016559"
}